{
  "gene_name": "Pyruvate kinase PKM",
  "term_label": "pyruvate kinase activity",
  "gene": "UniProtKB:P14618",
  "term_id": "GO:0004743",
  "gene_symbol": "PKM"
}